{
  "term_label": "Unknown molecular function",
  "gene_name": "Solute carrier family 41 member 1",
  "gene": "UniProtKB:Q8IVJ1",
  "term_id": "UNKNOWN:0001",
  "gene_symbol": "SLC41A1"
}